single-subunit type RNA polymerase binding [GO:0001050] (molecular function) Definition: Binding to a single subunit RNA polymerase enzyme, which is composed of a single catalytic subunit similar to the RNA polymerase enzymes from phages T3, T7, and SP6. Also known as: SP6-type RNA polymerase binding, T3-type RNA polymerase binding, T3/T7 type RNA polymerase binding, T7-type RNA polymerase binding Subtypes: mitochondrial single-subunit type RNA polymerase binding [GO:0001001], plastid single-subunit type RNA polymerase binding [GO:0001051] Relationships: is a type of GO:0070063 References: PMID:20701995 Sources: GOC:txnOH